{
  "term_id": "GO:0005886",
  "gene": "UniProtKB:Q6UXU4",
  "gene_symbol": "GSG1L",
  "term_label": "plasma membrane",
  "gene_name": "Germ cell-specific gene 1-like protein"
}